{
  "gene": "UniProtKB:Q13950",
  "term_label": "Unknown cellular component",
  "gene_name": "Runt-related transcription factor 2",
  "term_id": "UNKNOWN:0003",
  "gene_symbol": "RUNX2"
}